{
  "gene_symbol": "ROGDI",
  "gene_name": "Protein rogdi homolog",
  "term_id": "UNKNOWN:0002",
  "gene": "UniProtKB:Q9GZN7",
  "term_label": "Unknown biological process"
}